{
  "gene_symbol": "CHUK",
  "term_id": "GO:0033209",
  "gene": "UniProtKB:O15111",
  "term_label": "tumor necrosis factor-mediated signaling pathway",
  "gene_name": "Inhibitor of nuclear factor kappa-B kinase subunit alpha"
}